{
  "gene": "UniProtKB:Q9P2S2",
  "gene_symbol": "NRXN2",
  "term_id": "GO:0048787",
  "term_label": "presynaptic active zone membrane",
  "gene_name": "Neurexin-2"
}